positive regulation of renal phosphate excretion [GO:1903404] (biological process) Also known as: positive regulation of renal phosphate ion excretion, up regulation of renal phosphate excretion, up regulation of renal phosphate ion excretion, up-regulation of renal phosphate excretion, up-regulation of renal phosphate ion excretion, upregulation of renal phosphate excretion, upregulation of renal phosphate ion excretion, activation of renal phosphate excretion, activation of renal phosphate ion excretion Relationships: is a type of positive regulation of multicellular organismal process [GO:0051240]; is a type of regulation of renal phosphate excretion [GO:1903402]; positively regulates renal phosphate excretion [GO:0044722] Definition: Any process that activates or increases the frequency, rate or extent of renal phosphate excretion. References: PMID:8700837 Sources: GOC:TermGenie, GOC:pm, GO_REF:0000058